{
  "gene_name": "Homeobox protein Hox-D9",
  "gene": "UniProtKB:P28356",
  "term_label": "RNA polymerase II cis-regulatory region sequence-specific DNA binding",
  "term_id": "GO:0000978",
  "gene_symbol": "HOXD9"
}